{
  "term_label": "transcription regulator complex",
  "gene_name": "G protein pathway suppressor 2",
  "gene_symbol": "GPS2",
  "gene": "UniProtKB:Q13227",
  "term_id": "GO:0005667"
}